{
  "gene": "UniProtKB:Q02252",
  "gene_symbol": "ALDH6A1",
  "term_label": "methylmalonate-semialdehyde dehydrogenase (acylating, NAD) activity",
  "term_id": "GO:0004491",
  "gene_name": "Methylmalonate-semialdehyde dehydrogenase [acylating], mitochondrial"
}